beta-endorphin receptor activity [GO:0004979] (molecular function) Also known as: mu-opioid receptor activity Definition: Combining with beta-endorphin, and transmitting the signal across the membrane by activating an associated G-protein. Beta-endorphin is a peptide, 31 amino acids long, resulting from processing of the precursor proopiomelanocortin (POMC). Sources: GOC:ai, GOC:bf, Wikipedia:Beta-endorphin Relationships: is a type of melanocortin receptor activity [GO:0004977]; is a type of G protein-coupled opioid receptor activity [GO:0004985]; is a type of GO:0008188; has part beta-endorphin binding [GO:0031626]